{
  "term_label": "DNA replication factor C complex",
  "gene_name": "Replication factor C subunit 2",
  "term_id": "GO:0005663",
  "gene_symbol": "RFC2",
  "gene": "UniProtKB:P35250"
}